negative regulation of formation of translation initiation ternary complex [GO:1901191] (BP) Relationships: is a type of negative regulation of protein-containing complex assembly [GO:0031333]; is a type of GO:0045947; is a type of GO:1901190; RO_0002212 formation of translation initiation ternary complex [GO:0001677] Also known as: down regulation of formation of translation initiation ternary complex, down regulation of translation initiation ternary complex assembly, down-regulation of formation of translation initiation ternary complex, down-regulation of translation initiation ternary complex assembly, downregulation of formation of translation initiation ternary complex, downregulation of translation initiation ternary complex assembly, inhibition of translation initiation ternary complex assembly, negative regulation of translation initiation ternary complex assembly, inhibition of formation of translation initiation ternary complex Sources: GOC:TermGenie Definition: Any process that stops, prevents or reduces the frequency, rate or extent of formation of translation initiation ternary complex.